{
  "gene": "UniProtKB:Q03828",
  "term_label": "DNA-binding transcription factor activity, RNA polymerase II-specific",
  "gene_symbol": "EVX2",
  "term_id": "GO:0000981",
  "gene_name": "Homeobox even-skipped homolog protein 2"
}